positive regulation of B cell mediated immunity [GO:0002714] (biological process) Relationships: is a type of GO:0002708; is a type of GO:0002712; is a type of positive regulation of adaptive immune response based on somatic recombination of immune receptors built from immunoglobulin superfamily domains [GO:0002824]; positively regulates B cell mediated immunity [GO:0019724] Also known as: positive regulation of B lymphocyte mediated immunity, positive regulation of B-cell mediated immunity, positive regulation of B-lymphocyte mediated immunity, up regulation of B cell mediated immunity, up-regulation of B cell mediated immunity, upregulation of B cell mediated immunity, activation of B cell mediated immunity, stimulation of B cell mediated immunity Sources: GOC:add Definition: Any process that activates or increases the frequency, rate, or extent of B cell mediated immunity. Subtypes: positive regulation of B cell cytokine production [GO:0002723], positive regulation of immunoglobulin mediated immune response [GO:0002891], positive regulation of peripheral B cell deletion [GO:0002910], positive regulation of peripheral B cell anergy [GO:0002919], helper T cell enhancement of B cell mediated immune response [GO:0035399]